{
  "term_label": "adenylate cyclase-inhibiting G protein-coupled receptor signaling pathway",
  "term_id": "GO:0007193",
  "gene": "UniProtKB:Q6NUJ1",
  "gene_name": "Proactivator polypeptide-like 1",
  "gene_symbol": "PSAPL1"
}